coproporphyrinogen dehydrogenase activity [GO:0051989] (molecular function) Relationships: is_a oxidoreductase activity, acting on the CH-CH group of donors [GO:0016627] Definition: Catalysis of the reaction: coproporphyrinogen III + 2 S-adenosyl-L-methionine = protoporphyrinogen IX + 2 CO2 + 2 L-methionine + 2 5'-deoxyadenosine. Sources: EC:1.3.98.3 Also known as: oxygen-independent coproporphyrinogen-III oxidase activity, HemN, coproporphyrinogen III oxidase activity, coproporphyrinogen-III:S-adenosyl-L-methionine oxidoreductase (decarboxylating), radical SAM enzyme activity